{
  "term_id": "GO:0042113",
  "gene": "UniProtKB:Q8NDB2",
  "gene_symbol": "BANK1",
  "term_label": "B cell activation",
  "gene_name": "B-cell scaffold protein with ankyrin repeats"
}